protein transport out of membrane raft [GO:0032599] (biological process) Subtypes: chemokine receptor transport out of membrane raft [GO:0032600], protein transport out of plasma membrane raft [GO:0044862] Sources: GOC:mah Also known as: protein translocation out of membrane raft, protein transport out of lipid raft, receptor translocation out of membrane raft, receptor transport out of membrane raft Relationships: is a type of GO:0032594 Definition: The directed movement of a protein out of a membrane raft. Membrane rafts are small (10-200 nm), heterogeneous, highly dynamic, sterol- and sphingolipid-enriched membrane domains that compartmentalize cellular processes.